basic amino acid transmembrane import into vacuole [GO:0034490] (biological process) Sources: GOC:mah Definition: The directed movement of basic amino acids into the vacuole across the vacuolar membrane. Relationships: is a type of GO:0032975; is a type of GO:1990822 Subtypes: GO:0090513, L-lysine transmembrane import into vacuole [GO:0090517], L-arginine transmembrane import into vacuole [GO:0090518]